{
  "gene_name": "Transcription factor 15",
  "gene_symbol": "TCF15",
  "term_label": "RNA polymerase II transcription regulatory region sequence-specific DNA binding",
  "term_id": "GO:0000977",
  "gene": "UniProtKB:Q12870"
}